succinyldiaminopimelate transaminase activity [GO:0009016] (molecular function) Also known as: succinyldiaminopimelate aminotransferase activity, N-succinyl-L-2,6-diaminoheptanedioate:2-oxoglutarate aminotransferase activity, N-succinyl-L-diaminopimelic glutamic transaminase activity, succinyldiaminopimelate transferase activity Relationships: is a type of transaminase activity [GO:0008483] Sources: EC:2.6.1.17, RHEA:11960 Definition: Catalysis of the reaction: 2-oxoglutarate + N-succinyl-LL-2,6-diaminopimelate = L-2-succinylamino-6-oxopimelate + L-glutamate.